{
  "gene_name": "POM121-like protein 12",
  "term_id": "UNKNOWN:0003",
  "term_label": "Unknown cellular component",
  "gene": "UniProtKB:Q8N7R1",
  "gene_symbol": "POM121L12"
}